{
  "term_label": "regulation of transcription by RNA polymerase II",
  "gene": "UniProtKB:Q9H0M5",
  "term_id": "GO:0006357",
  "gene_symbol": "ZNF700",
  "gene_name": "Zinc finger protein 700"
}